oxidoreductase activity, acting on NAD(P)H [GO:0016651] (molecular function) Also known as: NAD(P)H dehydrogenase, oxidoreductase activity, acting on NADH or NADPH, other acceptor, oxidoreductase activity, acting on NADH or NADPH Definition: Catalysis of an oxidation-reduction (redox) reaction in which NADH or NADPH acts as a hydrogen or electron donor and reduces a hydrogen or electron acceptor. Subtypes: NADH dehydrogenase activity [GO:0003954], NADPH dehydrogenase activity [GO:0003959], oxidoreductase activity, acting on NAD(P)H as acceptor [GO:0016652], oxidoreductase activity, acting on NAD(P)H, heme protein as acceptor [GO:0016653], oxidoreductase activity, acting on NAD(P)H, quinone or similar compound as acceptor [GO:0016655], ferulate 5-hydroxylase activity [GO:0046424], oxidoreductase activity, acting on NAD(P)H, oxygen as acceptor [GO:0050664], selenite reductase (NADPH) activity [GO:0098623], GO:0098624, methylselenol reductase activity [GO:0098625], methylseleninic acid reductase activity [GO:0098626] Sources: GOC:ai Relationships: is a type of oxidoreductase activity [GO:0016491]